protein folding chaperone [GO:0044183] (molecular function) Definition: Binding to a protein or a protein-containing complex to assist the protein folding process. Also known as: chaperone activity, protein binding involved in protein folding Subtypes: ATP-dependent protein folding chaperone [GO:0140662] Relationships: is a type of molecular_function [GO:0003674]; is part of protein folding [GO:0006457]; has part unfolded protein binding [GO:0051082] Sources: GOC:mtg_cambridge_2009